{
  "gene_name": "Tissue-resident T-cell transcription regulator protein ZNF683",
  "gene_symbol": "ZNF683",
  "term_label": "DNA-binding transcription factor activity",
  "term_id": "GO:0003700",
  "gene": "UniProtKB:Q8IZ20"
}